{
  "term_label": "innate immune response",
  "gene_name": "E3 ubiquitin-protein ligase TRIM35",
  "gene_symbol": "TRIM35",
  "gene": "UniProtKB:Q9UPQ4",
  "term_id": "GO:0045087"
}